{
  "term_id": "GO:0005737",
  "gene": "UniProtKB:Q9UPT6",
  "term_label": "cytoplasm",
  "gene_symbol": "MAPK8IP3",
  "gene_name": "C-Jun-amino-terminal kinase-interacting protein 3"
}